{
  "gene_symbol": "HCN4",
  "term_id": "GO:0030424",
  "term_label": "axon",
  "gene_name": "Potassium_sodium hyperpolarization-activated cyclic nucleotide-gated channel 4",
  "gene": "UniProtKB:Q9Y3Q4"
}